{
  "term_label": "ubiquitin-protein transferase activity",
  "gene": "UniProtKB:Q96G75",
  "gene_name": "E3 ubiquitin-protein transferase RMND5B",
  "term_id": "GO:0004842",
  "gene_symbol": "RMND5B"
}